{
  "gene_name": "Casein kinase I isoform gamma-3",
  "term_id": "GO:0004674",
  "gene_symbol": "CSNK1G3",
  "gene": "UniProtKB:Q9Y6M4",
  "term_label": "protein serine/threonine kinase activity"
}